{
  "term_id": "GO:0043194",
  "gene_symbol": "NAV1",
  "term_label": "axon initial segment",
  "gene": "UniProtKB:Q8NEY1",
  "gene_name": "Neuron navigator 1"
}